{
  "gene_symbol": "EZR",
  "gene": "UniProtKB:P15311",
  "gene_name": "Ezrin",
  "term_id": "GO:0005912",
  "term_label": "adherens junction"
}